{
  "gene_name": "Alpha-actinin-3",
  "term_id": "GO:0030036",
  "term_label": "actin cytoskeleton organization",
  "gene_symbol": "ACTN3",
  "gene": "UniProtKB:Q08043"
}